cellular response to viscosity [GO:0097715] (biological process) Relationships: is a type of GO:0071214; is_a response to viscosity [GO:0097714] Definition: Any process that results in a change in state or activity of a cell (in terms of movement, secretion, enzyme production, gene expression, etc.) as a result of a viscosity stimulus. References: PMID:7061416 Sources: GOC:sl